{
  "gene_symbol": "WASF3",
  "term_id": "GO:2000601",
  "term_label": "positive regulation of Arp2/3 complex-mediated actin nucleation",
  "gene": "UniProtKB:Q9UPY6",
  "gene_name": "Actin-binding protein WASF3"
}